G protein-coupled acetylcholine receptor activity [GO:0016907] (molecular function) Definition: Combining with acetylcholine and transmitting the signal across the membrane by activating an associated G-protein; promotes the exchange of GDP for GTP on the alpha subunit of a heterotrimeric G-protein complex. Sources: GOC:bf, GOC:fj, GOC:mah Also known as: G protein coupled acetylcholine receptor activity, G-protein coupled acetylcholine receptor activity, acetylcholine receptor activity, G-protein coupled, metabotropic acetylcholine receptor activity, muscarinic acetylcholine receptor activity Relationships: is a type of GO:0008227; is a type of acetylcholine receptor activity [GO:0015464]; is a type of G protein-coupled neurotransmitter receptor activity [GO:0099528]; is part of GO:0007213